{
  "gene_symbol": "CFI",
  "term_label": "protein processing",
  "gene_name": "Complement factor I",
  "term_id": "GO:0016485",
  "gene": "UniProtKB:P05156"
}